{
  "gene_symbol": "CAMK2D",
  "gene": "UniProtKB:Q13557",
  "term_label": "neuron projection",
  "term_id": "GO:0043005",
  "gene_name": "Calcium_calmodulin-dependent protein kinase type II subunit delta"
}